{
  "gene_symbol": "WNT1",
  "term_id": "GO:0005109",
  "gene": "UniProtKB:P04628",
  "term_label": "frizzled binding",
  "gene_name": "Proto-oncogene Wnt-1"
}